lipid tube assembly [GO:0060988] (biological process) Also known as: lipid tubulation Relationships: is a type of GO:0065005 Subtypes: GO:0060989, lipid tube assembly involved in organelle fission [GO:0060990] Sources: GOC:ascb_2009, GOC:dph, GOC:tb Definition: The aggregation, arrangement and bonding together of a set of macromolecules to form a macromolecular complex that contains a tube of lipid surrounded by a protein coat involved in membrane shaping of vesicle membranes as they fuse or undergo fission.